{
  "term_label": "positive regulation of protein catabolic process",
  "gene_symbol": "ASB9",
  "term_id": "GO:0045732",
  "gene": "UniProtKB:Q96DX5",
  "gene_name": "Ankyrin repeat and SOCS box protein 9"
}